{
  "gene_name": "[Pyruvate dehydrogenase (acetyl-transferring)] kinase isozyme 3, mitochondrial",
  "term_id": "GO:0010510",
  "gene": "UniProtKB:Q15120",
  "term_label": "regulation of pyruvate decarboxylation to acetyl-CoA",
  "gene_symbol": "PDK3"
}